{
  "term_id": "GO:0005886",
  "gene_name": "Glutamate receptor 3",
  "term_label": "plasma membrane",
  "gene_symbol": "GRIA3",
  "gene": "UniProtKB:P42263"
}